{
  "gene_symbol": "ZNF513",
  "term_label": "transcription cis-regulatory region binding",
  "gene": "UniProtKB:Q8N8E2",
  "term_id": "GO:0000976",
  "gene_name": "Zinc finger protein 513"
}